{
  "term_id": "GO:0005879",
  "gene_name": "EF-hand domain-containing family member C2",
  "term_label": "axonemal microtubule",
  "gene": "UniProtKB:Q5JST6",
  "gene_symbol": "EFHC2"
}